4-aminobenzoate 1-monooxygenase activity [GO:0018670] (MF) Definition: Catalysis of the reaction: 4-aminobenzoate + NADPH + H+ + O2 = 4-hydroxyaniline + NADP+ + H2O + CO2. Also known as: 4-aminobenzoate hydroxylase activity, 4-aminobenzoate dehydrogenase activity, 4-aminobenzoate monooxygenase activity, 4-aminobenzoate,NAD(P)H:oxygen oxidoreductase (1-hydroxylating, decarboxylating) Sources: EC:1.14.13.27 Relationships: is a type of oxidoreductase activity, acting on paired donors, with incorporation or reduction of molecular oxygen, NAD(P)H as one donor, and incorporation of one atom of oxygen [GO:0016709]